{
  "gene_symbol": "WBP2NL",
  "gene": "UniProtKB:Q6ICG8",
  "term_id": "GO:0045893",
  "gene_name": "Postacrosomal sheath WW domain-binding protein",
  "term_label": "positive regulation of DNA-templated transcription"
}